{
  "term_id": "GO:0009143",
  "term_label": "nucleoside triphosphate catabolic process",
  "gene_name": "Inosine triphosphate pyrophosphatase",
  "gene": "UniProtKB:Q9BY32",
  "gene_symbol": "ITPA"
}